positive regulation of type I interferon-mediated signaling pathway [GO:0060340] (biological process) Sources: GOC:dph Relationships: is a type of positive regulation of cytokine-mediated signaling pathway [GO:0001961]; is a type of GO:0045089; is a type of regulation of type I interferon-mediated signaling pathway [GO:0060338]; positively regulates type I interferon-mediated signaling pathway [GO:0060337] Also known as: positive regulation of type I interferon-mediated signalling pathway Definition: Any process that increases the rate, frequency or extent of a type I interferon-mediated signaling pathway.